maintenance of transcriptional fidelity during transcription elongation by RNA polymerase III [GO:0001195] (biological process) Definition: Suppression of the occurrence of transcriptional errors, such as substitutions and/or insertions of nucleotides that do not correctly match the template base, during the process of transcription elongation from a RNA polymerase III promoter. Also known as: maintenance of transcriptional fidelity during DNA-dependent transcription elongation from RNA polymerase III promoter, maintenance of transcriptional fidelity during DNA-templated transcription elongation from RNA polymerase III promoter Relationships: is a type of maintenance of transcriptional fidelity during transcription elongation [GO:0001192]; is part of transcription elongation by RNA polymerase III [GO:0006385] Sources: GOC:txnOH